{
  "gene_symbol": "SLC7A1",
  "term_id": "GO:0097638",
  "gene": "UniProtKB:P30825",
  "term_label": "L-arginine import across plasma membrane",
  "gene_name": "High affinity cationic amino acid transporter 1"
}